sarcoplasmic reticulum calcium ion transport [GO:0070296] (biological process) Sources: GOC:BHF, GOC:vk Definition: The directed movement of calcium ions (Ca2+) into, out of or within the sarcoplasmic reticulum. Relationships: is a type of calcium ion transport [GO:0006816] Subtypes: release of sequestered calcium ion into cytosol by sarcoplasmic reticulum [GO:0014808], calcium ion import into sarcoplasmic reticulum [GO:1990036]